{
  "term_label": "mitochondrial matrix",
  "gene_name": "Glutaredoxin-related protein 5, mitochondrial",
  "gene_symbol": "GLRX5",
  "term_id": "GO:0005759",
  "gene": "UniProtKB:Q86SX6"
}